{
  "gene_symbol": "CDV3",
  "gene": "UniProtKB:Q9UKY7",
  "gene_name": "Protein CDV3 homolog",
  "term_id": "GO:0005737",
  "term_label": "cytoplasm"
}